regulation of uracil import across plasma membrane [GO:1905529] (biological process) Relationships: is_a regulation of transmembrane transport [GO:0034762]; regulates uracil import across plasma membrane [GO:0098721] Subtypes: negative regulation of uracil import across plasma membrane [GO:1905530], positive regulation of uracil import across plasma membrane [GO:1905531] References: PMID:26536126 Sources: GOC:TermGenie, GO_REF:0000058 Definition: Any process that modulates the frequency, rate or extent of uracil import across plasma membrane.